{
  "gene_name": "Deoxyribose-phosphate aldolase",
  "gene": "UniProtKB:Q9Y315",
  "term_id": "GO:0004139",
  "gene_symbol": "DERA",
  "term_label": "deoxyribose-phosphate aldolase activity"
}